{
  "gene_symbol": "TRNP1",
  "term_id": "GO:0003677",
  "gene_name": "TMF-regulated nuclear protein 1",
  "term_label": "DNA binding",
  "gene": "UniProtKB:Q6NT89"
}